{
  "gene_name": "Testis-specific Y-encoded-like protein 6",
  "term_label": "chromatin binding",
  "gene": "UniProtKB:Q8N831",
  "gene_symbol": "TSPYL6",
  "term_id": "GO:0003682"
}